{
  "term_id": "GO:0031710",
  "term_label": "neuromedin B receptor binding",
  "gene_name": "Neuromedin-B",
  "gene": "UniProtKB:P08949",
  "gene_symbol": "NMB"
}